{
  "term_id": "GO:0007189",
  "gene_name": "Adenylate cyclase type 1",
  "term_label": "adenylate cyclase-activating G protein-coupled receptor signaling pathway",
  "gene": "UniProtKB:Q08828",
  "gene_symbol": "ADCY1"
}